{
  "gene": "UniProtKB:Q8TCJ0",
  "gene_symbol": "FBXO25",
  "term_label": "nucleus",
  "term_id": "GO:0005634",
  "gene_name": "F-box only protein 25"
}